dCTP deaminase activity [GO:0008829] (molecular function) Sources: EC:3.5.4.13 Definition: Catalysis of the reaction: dCTP + H2O = dUTP + NH3. Also known as: 5-methyl-dCTP deaminase activity, dCTP aminohydrolase activity, deoxycytidine triphosphate deaminase activity Relationships: is_a hydrolase activity, acting on carbon-nitrogen (but not peptide) bonds, in cyclic amidines [GO:0016814]; is_a deaminase activity [GO:0019239]